(+)-secoisolariciresinol catabolic process [GO:1902134] (biological process) References: PMID:15949826, PMID:9872995 Sources: GOC:TermGenie Also known as: (+)-secoisolariciresinol breakdown, (+)-secoisolariciresinol catabolism, (+)-secoisolariciresinol degradation Relationships: is a type of phenol-containing compound catabolic process [GO:0019336]; is a type of diol catabolic process [GO:0034313]; is a type of lignan catabolic process [GO:0046273] Definition: The chemical reactions and pathways resulting in the breakdown of (+)-secoisolariciresinol.